{
  "gene_name": "E3 ubiquitin-protein ligase UBR2",
  "gene_symbol": "UBR2",
  "term_id": "GO:0071596",
  "term_label": "ubiquitin-dependent protein catabolic process via the N-end rule pathway",
  "gene": "UniProtKB:Q8IWV8"
}